1,3-beta-oligoglucan phosphorylase activity [GO:0047515] (molecular function) Relationships: is a type of hexosyltransferase activity [GO:0016758] Also known as: 1,3-beta-D-oligoglucan:phosphate alpha-D-glucosyltransferase activity, beta-1,3-oligoglucan phosphorylase activity, beta-1,3-oligoglucan:orthophosphate glucosyltransferase II activity Sources: EC:2.4.1.30, MetaCyc:13-BETA-OLIGOGLUCAN-PHOSPHORYLASE-RXN Definition: Catalysis of the reaction: [oligomeric (1->3)-beta-D-glucosyl](n) + phosphate = [(1->3)-beta-D-glucosyl](n-1) + alpha-D-glucose 1-phosphate.